{
  "gene": "UniProtKB:Q7Z3F1",
  "term_id": "GO:0030514",
  "gene_symbol": "GPR155",
  "gene_name": "Integral membrane protein GPR155",
  "term_label": "negative regulation of BMP signaling pathway"
}